{
  "term_id": "GO:0003735",
  "gene_symbol": "RPL39L",
  "term_label": "structural constituent of ribosome",
  "gene": "UniProtKB:Q96EH5",
  "gene_name": "Ribosomal protein eL39-like 2"
}